{
  "gene_symbol": "OSGIN2",
  "term_id": "UNKNOWN:0003",
  "term_label": "Unknown cellular component",
  "gene": "UniProtKB:Q9Y236",
  "gene_name": "Oxidative stress-induced growth inhibitor 2"
}